{
  "term_label": "Unknown cellular component",
  "gene_name": "Mucin-7",
  "term_id": "UNKNOWN:0003",
  "gene_symbol": "MUC7",
  "gene": "UniProtKB:Q8TAX7"
}